{
  "gene_symbol": "BRF1",
  "term_label": "nucleus",
  "gene": "UniProtKB:Q92994",
  "term_id": "GO:0005634",
  "gene_name": "Transcription factor IIIB 90 kDa subunit"
}